{
  "gene_name": "Deuterosome assembly protein 1",
  "gene_symbol": "DEUP1",
  "gene": "UniProtKB:Q05D60",
  "term_id": "UNKNOWN:0001",
  "term_label": "Unknown molecular function"
}